{
  "gene_symbol": "CHSY3",
  "term_label": "chondroitin sulfate proteoglycan biosynthetic process",
  "gene_name": "Chondroitin sulfate synthase 3",
  "gene": "UniProtKB:Q70JA7",
  "term_id": "GO:0050650"
}